{
  "gene_name": "Cation channel sperm-associated auxiliary subunit gamma",
  "term_id": "UNKNOWN:0001",
  "term_label": "Unknown molecular function",
  "gene": "UniProtKB:Q6ZRH7",
  "gene_symbol": "CATSPERG"
}